ASAP complex [GO:0061574] (cellular component) Relationships: is a type of protein-containing complex [GO:0032991] Definition: A protein complex involved in regulation of mRNA processing and apoptosis. It binds to RNA in a sequence-independent manner and is recruited to the EJC prior to or during the splicing process. In humans the core proteins are RNPS1, SAP18 and ACIN1. References: PMID:12665594, PMID:16314458, PMID:22388736 Sources: GOC:dph